{
  "term_label": "calcineurin-NFAT signaling cascade",
  "gene_symbol": "NFATC1",
  "gene_name": "Nuclear factor of activated T-cells, cytoplasmic 1",
  "term_id": "GO:0033173",
  "gene": "UniProtKB:O95644"
}